xenobiotic transport across blood-nerve barrier [GO:0061772] (biological process) References: PMID:22733753 Sources: GOC:dph Definition: The directed movement of a xenobiotic through the blood-nerve barrier. Relationships: is a type of xenobiotic transport [GO:0042908] Also known as: drug transport across perineurial barrier, drug transport across blood-nerve barrier